{
  "gene": "UniProtKB:P0DN77",
  "term_id": "GO:0016038",
  "gene_symbol": "OPN1MW2",
  "term_label": "absorption of visible light",
  "gene_name": "Medium-wave-sensitive opsin 2"
}